regulation of removal of superoxide radicals [GO:2000121] (biological process) Definition: Any process that modulates the frequency, rate or extent of removal of superoxide radicals. Subtypes: negative regulation of removal of superoxide radicals [GO:1904832], positive regulation of removal of superoxide radicals [GO:1904833] Sources: GOC:obol Relationships: is_a GO:0090322; is a type of GO:1900407; is a type of regulation of response to reactive oxygen species [GO:1901031]; RO_0002211 removal of superoxide radicals [GO:0019430] Also known as: regulation of removal of O2-, regulation of removal of oxygen free radicals